{
  "gene_name": "Vacuolar ATPase assembly integral membrane protein VMA21",
  "term_label": "vacuolar proton-transporting V-type ATPase complex assembly",
  "gene": "UniProtKB:Q3ZAQ7",
  "gene_symbol": "VMA21",
  "term_id": "GO:0070072"
}